{
  "gene_symbol": "OR2W6P",
  "term_id": "GO:0004984",
  "term_label": "olfactory receptor activity",
  "gene": "UniProtKB:Q8NHA6",
  "gene_name": "Putative olfactory receptor 2W6"
}